blood coagulation, common pathway [GO:0072377] (biological process) Relationships: is a type of GO:0072376; is part of GO:0072378 Definition: A protein activation cascade that contributes to blood coagulation and consists of events leading from the formation of activated Factor Xa by either the intrinsic or extrinsic pathway, to the formation of active thrombin, the cleavage of fibrinogen by thrombin, and the formation of cleaved fibrin into a stable multimeric, cross-linked complex. Note: See also the biological process term 'blood coagulation, intrinsic pathway ; GO:0007597'. Regulation: regulated by regulation of blood coagulation, common pathway [GO:2000260]; negatively regulated by GO:2000261; positively regulated by positive regulation of blood coagulation, common pathway [GO:2000262] References: PMID:1931959 Sources: GOC:add, GOC:mah, GOC:pde